{
  "gene": "UniProtKB:P42229",
  "term_id": "GO:0060397",
  "gene_symbol": "STAT5A",
  "term_label": "growth hormone receptor signaling pathway via JAK-STAT",
  "gene_name": "Signal transducer and activator of transcription 5A"
}